{
  "gene": "UniProtKB:P22760",
  "term_label": "endoplasmic reticulum membrane",
  "term_id": "GO:0005789",
  "gene_symbol": "AADAC",
  "gene_name": "Arylacetamide deacetylase"
}